{
  "gene_name": "One cut domain family member 2",
  "term_label": "regulation of transcription by RNA polymerase II",
  "term_id": "GO:0006357",
  "gene_symbol": "ONECUT2",
  "gene": "UniProtKB:O95948"
}